DASH complex [GO:0042729] (cellular component) Note: Note that this complex is conserved in fungi but has not been observed in metazoans. Definition: A large protein complex, containing around 8-10 subunits in yeast, including Duo1p, Dam1p, Dad1p and Ask1p. The complex forms part of the outer kinetochore, associates with microtubules when the kinetochore attaches to the spindle, and plays a role in spindle attachment, chromosome segregation and spindle stability. Relationships: is a type of nuclear protein-containing complex [GO:0140513]; is part of outer kinetochore [GO:0000940] References: PMID:11782438, PMID:11799062, PMID:15632076, PMID:15640796 Sources: GOC:jl, GOC:vw Also known as: DDD complex, Dam1 complex, Duo1p-Dam1p-Dad1p complex, condensed nuclear chromosome kinetochore-associated DASH complex